{
  "term_label": "spermatid development",
  "gene_name": "Coiled-coil domain-containing protein 42",
  "gene": "UniProtKB:Q96M95",
  "gene_symbol": "CCDC42",
  "term_id": "GO:0007286"
}